negative regulation of juvenile hormone secretion [GO:0045972] (biological process) Relationships: is a type of GO:0007558; is a type of negative regulation of lipid transport [GO:0032369]; is a type of GO:0046888; is a type of GO:0051241; negatively regulates juvenile hormone secretion [GO:0045443] Definition: Any process that stops, prevents, or reduces the frequency, rate or extent of the regulated release of juvenile hormone. Also known as: down regulation of juvenile hormone secretion, down-regulation of juvenile hormone secretion, downregulation of juvenile hormone secretion, inhibition of juvenile hormone secretion Sources: GOC:go_curators